{
  "gene": "UniProtKB:P49758",
  "term_id": "GO:0043005",
  "term_label": "neuron projection",
  "gene_name": "Regulator of G-protein signaling 6",
  "gene_symbol": "RGS6"
}